metal-dependent deNEDDylase activity [GO:0140758] (MF) References: PMID:25628956 Relationships: is a type of metallopeptidase activity [GO:0008237]; is a type of deNEDDylase activity [GO:0019784] Definition: An metal-dependent isopeptidase activity that cleaves NEDD8 from a target protein to which it is conjugated.